{
  "gene_symbol": "SLC48A1",
  "term_id": "GO:0015886",
  "gene": "UniProtKB:Q6P1K1",
  "gene_name": "Heme transporter HRG1",
  "term_label": "heme transport"
}